cellular response to nerve growth factor stimulus [GO:1990090] (biological process) Subtypes: cellular response to brain-derived neurotrophic factor stimulus [GO:1990416] Definition: A process that results in a change in state or activity of a cell (in terms of movement, secretion, enzyme production, gene expression, etc.) as a result of a nerve growth factor stimulus. Relationships: is a type of cellular response to growth factor stimulus [GO:0071363]; is a type of GO:1990089 Also known as: cellular response to NGF References: PMID:22399805 Sources: Wikipedia:Nerve_growth_factor